positive regulation of transcription by RNA polymerase V [GO:1904281] (BP) References: PMID:24726328 Sources: GOC:TermGenie, GO_REF:0000058 Relationships: is a type of GO:0045893; is a type of regulation of transcription by RNA polymerase V [GO:1904279]; positively regulates GO:0001060 Also known as: positive regulation of transcription from RNA pol V promoter, positive regulation of transcription from RNA polymerase V promoter, up regulation of transcription from RNA pol V promoter, up regulation of transcription from RNA polymerase V promoter, up-regulation of transcription from RNA pol V promoter, up-regulation of transcription from RNA polymerase V promoter, upregulation of transcription from RNA pol V promoter, upregulation of transcription from RNA polymerase V promoter, activation of transcription from RNA pol V promoter, activation of transcription from RNA polymerase V promoter Definition: Any process that activates or increases the frequency, rate or extent of transcription mediated by RNA polymerase V.